{
  "term_id": "GO:0046961",
  "gene": "UniProtKB:Q93050",
  "gene_symbol": "ATP6V0A1",
  "gene_name": "V-type proton ATPase 116 kDa subunit a 1",
  "term_label": "proton-transporting ATPase activity, rotational mechanism"
}